regulation of 18-methylnonadec-1-ene biosynthetic process [GO:1900950] (biological process) Sources: GOC:TermGenie, GOC:mengo_curators Relationships: is a type of regulation of olefin biosynthetic process [GO:1900911]; regulates GO:1900881 Subtypes: GO:1900951, GO:1900952 Also known as: regulation of 18-methylnonadec-1-ene anabolism, regulation of 18-methylnonadec-1-ene biosynthesis, regulation of 18-methylnonadec-1-ene formation, regulation of 18-methylnonadec-1-ene synthesis Definition: Any process that modulates the frequency, rate or extent of 18-methylnonadec-1-ene biosynthetic process.